{
  "gene": "UniProtKB:P51449",
  "term_label": "RNA polymerase II cis-regulatory region sequence-specific DNA binding",
  "gene_name": "Nuclear receptor ROR-gamma",
  "gene_symbol": "RORC",
  "term_id": "GO:0000978"
}